{
  "gene": "UniProtKB:Q16651",
  "gene_symbol": "PRSS8",
  "gene_name": "Prostasin",
  "term_label": "serine-type peptidase activity",
  "term_id": "GO:0008236"
}